{
  "gene_name": "Cadherin-2",
  "gene_symbol": "CDH2",
  "term_id": "GO:0005737",
  "gene": "UniProtKB:P19022",
  "term_label": "cytoplasm"
}